{
  "term_id": "GO:0043005",
  "term_label": "neuron projection",
  "gene": "UniProtKB:P32745",
  "gene_name": "Somatostatin receptor type 3",
  "gene_symbol": "SSTR3"
}